{
  "term_id": "GO:0005886",
  "term_label": "plasma membrane",
  "gene_symbol": "NPBWR1",
  "gene": "UniProtKB:P48145",
  "gene_name": "Neuropeptides B_W receptor type 1"
}